{
  "gene_symbol": "U2AF2",
  "gene": "UniProtKB:P26368",
  "gene_name": "Splicing factor U2AF 65 kDa subunit",
  "term_id": "GO:0071004",
  "term_label": "U2-type prespliceosome"
}